anthocyanin biosynthetic process involved in anthocyanin accumulation in response to UV light [GO:0043483] (biological process) Relationships: is a type of GO:0009718; is a type of pigment biosynthetic process involved in pigment accumulation [GO:0043477]; is part of anthocyanin accumulation in tissues in response to UV light [GO:0043481] Also known as: anthocyanin biosynthesis during anthocyanin accumulation in tissues in response to UV light stimulus, anthocyanin biosynthetic process during anthocyanin accumulation in response to UV light, anthocyanin biosynthetic process during anthocyanin accumulation in tissues in response to UV light stimulus Definition: The chemical reactions and pathways resulting in the formation of the pigment anthocyanin, contributing to anthocyanin accumulation in a tissue in response to a UV light stimulus. Sources: GOC:dph, GOC:jl, GOC:tb